2-hydroxy-6-oxo-6-phenylhexa-2,4-dienoate reductase activity [GO:0047118] (molecular function) Definition: Catalysis of the reaction: 2,6-dioxo-6-phenylhexanoate + NADP+ = 2-hydroxy-6-oxo-6-phenylhexa-2,4-dienoate + H+ + NADPH. Sources: EC:1.3.1.40, RHEA:24268 Relationships: is a type of oxidoreductase activity, acting on the CH-CH group of donors, NAD or NADP as acceptor [GO:0016628] Also known as: 2,6-dioxo-6-phenylhexanoate:NADP+ delta2-oxidoreductase activity, 2-hydroxy-6-oxo-phenylhexa-2,4-dienoate (reduced nicotinamide adenine dinucleotide phosphate) reductase activity